gravitaxis [GO:0042332] (BP) Relationships: is a type of response to gravity [GO:0009629]; is a type of GO:0042330 Definition: The directed movement of a motile cell or organism in response to gravity. Subtypes: GO:0048060, positive gravitaxis [GO:0048061] Sources: GOC:jid, GOC:jl Also known as: geotactic behavior, geotactic behaviour, geotaxis, gravitactic behavior, gravitactic behaviour, taxis in response to gravitational stimulus, taxis in response to gravity